{
  "gene_symbol": "IGKV1-6",
  "term_label": "immunoglobulin complex",
  "term_id": "GO:0019814",
  "gene": "UniProtKB:A0A0C4DH72",
  "gene_name": "Immunoglobulin kappa variable 1-6"
}